{
  "term_id": "UNKNOWN:0003",
  "term_label": "Unknown cellular component",
  "gene_symbol": "RNF141",
  "gene_name": "RING finger protein 141",
  "gene": "UniProtKB:Q8WVD5"
}